meiotic centromeric cohesion protection in anaphase I [GO:1990813] (biological process) Also known as: anaphase cohesion protection, protection of centromeric cohesion during meiotic anaphase I Relationships: is_a maintenance of meiotic sister chromatid cohesion, centromeric [GO:0035875]; is a type of meiotic cell cycle process [GO:1903046]; is part of GO:0045143 References: PMID:14730319, PMID:25533956 Definition: The process in which the association between sister chromatids of a replicated chromosome centromeric region is maintained during homologous chromosome segregation at meiotic anaphase I after cohesin is cleaved by separase along the arm regions.